3-dehydroshikimate dehydratase activity [GO:0046565] (molecular function) Sources: EC:4.2.1.118, MetaCyc:DHSHIKIMATE-DEHYDRO-RXN Definition: Catalysis of the reaction: 3-dehydroshikimate = 3,4-dihydroxybenzoate + H2O. 3,4-dihydroxybenzoate is also known as protocatechuate. Relationships: is a type of GO:0016836